{
  "gene": "UniProtKB:P17032",
  "gene_symbol": "ZNF37A",
  "term_id": "GO:0006357",
  "term_label": "regulation of transcription by RNA polymerase II",
  "gene_name": "Zinc finger protein 37A"
}